{
  "gene_symbol": "FAM107A",
  "term_id": "GO:0045202",
  "gene_name": "Actin-associated protein FAM107A",
  "term_label": "synapse",
  "gene": "UniProtKB:O95990"
}